{
  "term_label": "Unknown biological process",
  "gene": "UniProtKB:Q9BVM4",
  "term_id": "UNKNOWN:0002",
  "gene_name": "Gamma-glutamylaminecyclotransferase",
  "gene_symbol": "GGACT"
}